{
  "gene_symbol": "C9orf163",
  "gene_name": "Uncharacterized protein C9orf163",
  "term_id": "UNKNOWN:0002",
  "gene": "UniProtKB:Q8N9P6",
  "term_label": "Unknown biological process"
}